{
  "term_id": "UNKNOWN:0001",
  "gene": "UniProtKB:A0A075B6X3",
  "gene_name": "T cell receptor alpha joining 32 (Fragment)",
  "gene_symbol": "TRAJ32",
  "term_label": "Unknown molecular function"
}